{
  "term_label": "positive regulation of phosphatidylinositol 3-kinase/protein kinase B signal transduction",
  "gene_symbol": "PDGFA",
  "gene": "UniProtKB:P04085",
  "term_id": "GO:0051897",
  "gene_name": "Platelet-derived growth factor subunit A"
}